pyridoxal transport [GO:0031920] (biological process) Sources: GOC:mah Subtypes: pyridoxal transmembrane transport [GO:1903090] Relationships: is_a organic cation transport [GO:0015695]; is a type of organic hydroxy compound transport [GO:0015850]; is a type of vitamin B6 transport [GO:0031919] Definition: The directed movement of pyridoxal into, out of or within a cell, or between cells, by means of some agent such as a transporter or pore. Pyridoxal, 3-hydroxy-5-(hydroxymethyl)-2-methyl-4-pyridinecarboxaldehyde, is one of the vitamin B6 compounds. Pyridoxal, pyridoxamine and pyridoxine are collectively known as vitamin B6, and are efficiently converted to the biologically active form of vitamin B6, pyridoxal phosphate.